{
  "gene": "UniProtKB:Q14623",
  "gene_symbol": "IHH",
  "term_label": "cell fate specification",
  "gene_name": "Indian hedgehog protein",
  "term_id": "GO:0001708"
}